{
  "gene_symbol": "COL5A3",
  "term_label": "extracellular matrix",
  "gene": "UniProtKB:P25940",
  "gene_name": "Collagen alpha-3(V) chain",
  "term_id": "GO:0031012"
}